{
  "gene_symbol": "CHRNB4",
  "gene": "UniProtKB:P30926",
  "term_id": "GO:0034220",
  "gene_name": "Neuronal acetylcholine receptor subunit beta-4",
  "term_label": "monoatomic ion transmembrane transport"
}